{
  "term_label": "Unknown molecular function",
  "gene_symbol": "VWC2L",
  "gene_name": "von Willebrand factor C domain-containing protein 2-like",
  "gene": "UniProtKB:B2RUY7",
  "term_id": "UNKNOWN:0001"
}